{
  "gene_name": "Interleukin-12 receptor subunit beta-2",
  "gene": "UniProtKB:Q99665",
  "term_label": "positive regulation of cell population proliferation",
  "gene_symbol": "IL12RB2",
  "term_id": "GO:0008284"
}